{
  "term_id": "UNKNOWN:0001",
  "gene_symbol": "TRBV12-5",
  "gene": "UniProtKB:A0A1B0GX78",
  "term_label": "Unknown molecular function",
  "gene_name": "T cell receptor beta variable 12-5"
}